{
  "gene": "UniProtKB:Q9ULG6",
  "term_id": "UNKNOWN:0002",
  "gene_symbol": "CCPG1",
  "term_label": "Unknown biological process",
  "gene_name": "Cell cycle progression protein 1"
}